positive regulation of receptor internalization [GO:0002092] (biological process) Also known as: up regulation of receptor internalization, up-regulation of receptor internalization, upregulation of receptor internalization, activation of receptor internalization, stimulation of receptor internalization Sources: GOC:hjd Relationships: is a type of regulation of receptor internalization [GO:0002090]; is_a positive regulation of receptor-mediated endocytosis [GO:0048260]; positively regulates GO:0031623 Definition: Any process that activates or increases the frequency, rate or extent of receptor internalization. Subtypes: GO:1904022